regulation of SCF-dependent proteasomal ubiquitin-dependent protein catabolic process [GO:0062025] (biological process) References: PMID:28007894 Relationships: is a type of GO:0032434; regulates GO:0031146 Subtypes: negative regulation of SCF-dependent proteasomal ubiquitin-dependent catabolic process [GO:0062026], positive regulation of SCF-dependent proteasomal ubiquitin-dependent catabolic process [GO:0062027] Definition: Any process that modualtes the rate, frequency or extent of SCF-dependent proteasomal ubiquitin-dependent protein catabolic process, the chemical reactions and pathways resulting in the breakdown of a protein or peptide by hydrolysis of its peptide bonds, initiated by the covalent attachment of ubiquitin, with ubiquitin-protein ligation catalyzed by an SCF (Skp1/Cul1/F-box protein) complex, and mediated by the proteasome.